{
  "gene_name": "Olfactory receptor 4C15",
  "term_id": "GO:0004984",
  "gene": "UniProtKB:Q8NGM1",
  "term_label": "olfactory receptor activity",
  "gene_symbol": "OR4C15"
}